convergent extension involved in rhombomere morphogenesis [GO:1904125] (biological process) Regulation: regulated by regulation of convergent extension involved in rhombomere morphogenesis [GO:1904133]; negatively regulated by negative regulation of convergent extension involved in rhombomere morphogenesis [GO:1904134]; positively regulated by positive regulation of convergent extension involved in rhombomere morphogenesis [GO:1904135] Definition: Any convergent extension that is involved in rhombomere morphogenesis. References: PMID:24892953 Sources: GOC:TermGenie, GOC:dph, GO_REF:0000060 Relationships: is a type of convergent extension involved in gastrulation [GO:0060027]; is a type of convergent extension involved in organogenesis [GO:0060029]; is part of rhombomere morphogenesis [GO:0021593]